{
  "gene": "UniProtKB:P0DMP2",
  "gene_symbol": "SRGAP2B",
  "term_label": "nervous system development",
  "term_id": "GO:0007399",
  "gene_name": "SLIT-ROBO Rho GTPase-activating protein 2B"
}